{
  "gene_symbol": "MACF1",
  "term_id": "GO:0015629",
  "term_label": "actin cytoskeleton",
  "gene_name": "Microtubule-actin cross-linking factor 1, isoforms 1_2_3_4_5",
  "gene": "UniProtKB:Q9UPN3"
}